{
  "gene_name": "Probable G-protein coupled receptor 63",
  "gene_symbol": "GPR63",
  "term_label": "G protein-coupled receptor signaling pathway",
  "gene": "UniProtKB:Q9BZJ6",
  "term_id": "GO:0007186"
}